{
  "gene": "UniProtKB:Q16665",
  "term_label": "intracellular oxygen homeostasis",
  "term_id": "GO:0032364",
  "gene_name": "Hypoxia-inducible factor 1-alpha",
  "gene_symbol": "HIF1A"
}